myelin-proteolipid O-palmitoyltransferase activity [GO:0047157] (molecular function) Definition: Catalysis of the reaction: [myelin proteolipid] + palmityl-CoA = [myelin proteolipid] O-palmitoylprotein + CoA. Relationships: is a type of O-palmitoyltransferase activity [GO:0016416] Also known as: acyl-protein synthase activity, [myelin-proteolipid] O-palmitoyltransferase activity, myelin PLP acyltransferase activity, palmitoyl-CoA:[myelin-proteolipid] O-palmitoyltransferase activity References: PMID:3818589